{
  "gene_symbol": "IGHV3OR16-10",
  "gene": "UniProtKB:A0A075B7F0",
  "term_id": "UNKNOWN:0003",
  "term_label": "Unknown cellular component",
  "gene_name": "Immunoglobulin heavy variable 3_OR16-10 (non-functional) (Fragment)"
}